{
  "gene_name": "Bridging integrator 2",
  "gene_symbol": "BIN2",
  "term_label": "podosome assembly",
  "term_id": "GO:0071800",
  "gene": "UniProtKB:Q9UBW5"
}